{
  "gene": "UniProtKB:Q8WWM7",
  "term_label": "stress granule assembly",
  "term_id": "GO:0034063",
  "gene_symbol": "ATXN2L",
  "gene_name": "Ataxin-2-like protein"
}